{
  "term_label": "Unknown biological process",
  "term_id": "UNKNOWN:0002",
  "gene_symbol": "FBXW9",
  "gene": "UniProtKB:Q5XUX1",
  "gene_name": "F-box_WD repeat-containing protein 9"
}